{
  "term_label": "plasma membrane",
  "gene": "UniProtKB:Q0GE19",
  "term_id": "GO:0005886",
  "gene_name": "Sodium_bile acid cotransporter 7",
  "gene_symbol": "SLC10A7"
}